{
  "term_label": "Unknown biological process",
  "gene_name": "Inositol 1,4,5-trisphosphate receptor-interacting protein",
  "gene_symbol": "ITPRIP",
  "gene": "UniProtKB:Q8IWB1",
  "term_id": "UNKNOWN:0002"
}